{
  "gene_name": "C4b-binding protein alpha chain",
  "gene": "UniProtKB:P04003",
  "term_label": "Unknown molecular function",
  "term_id": "UNKNOWN:0001",
  "gene_symbol": "C4BPA"
}